{
  "gene_name": "Protein turtle homolog A",
  "gene_symbol": "IGSF9",
  "gene": "UniProtKB:Q9P2J2",
  "term_label": "plasma membrane",
  "term_id": "GO:0005886"
}